{
  "term_id": "GO:0030510",
  "gene": "UniProtKB:Q6MZW2",
  "gene_name": "Follistatin-related protein 4",
  "term_label": "regulation of BMP signaling pathway",
  "gene_symbol": "FSTL4"
}